{
  "gene_name": "Small integral membrane protein 9",
  "gene": "UniProtKB:A6NGZ8",
  "term_id": "UNKNOWN:0003",
  "gene_symbol": "SMIM9",
  "term_label": "Unknown cellular component"
}